peptidyl-threonine dephosphorylation [GO:0035970] (biological process) Sources: GOC:bf Relationships: is a type of protein dephosphorylation [GO:0006470] Definition: The removal of phosphoric residues from peptidyl-O-phospho-L-threonine to form peptidyl-threonine.